HOPS complex [GO:0030897] (cellular component) References: PMID:10944212, PMID:23645161 Relationships: is a type of membrane protein complex [GO:0098796]; is a type of vesicle tethering complex [GO:0099023] Definition: A multimeric protein complex that associates with the vacuolar membrane, late endosomal (multivesicular body) and lysosomal membranes. HOPS is a tethering complex involved in vesicle fusion. Subtypes: vacuolar HOPS complex [GO:1902500], multivesicular body HOPS complex [GO:1902502]